{
  "term_label": "regulation of transcription by RNA polymerase II",
  "term_id": "GO:0006357",
  "gene": "UniProtKB:Q9NSC2",
  "gene_symbol": "SALL1",
  "gene_name": "Sal-like protein 1"
}